{
  "term_label": "protein maturation",
  "gene_name": "Chymase",
  "gene": "UniProtKB:P23946",
  "gene_symbol": "CMA1",
  "term_id": "GO:0051604"
}